{
  "gene": "UniProtKB:Q9ULD6",
  "term_id": "GO:0005929",
  "gene_name": "Protein inturned",
  "gene_symbol": "INTU",
  "term_label": "cilium"
}